{
  "gene_symbol": "EPHA2",
  "gene": "UniProtKB:P29317",
  "term_label": "plasma membrane",
  "gene_name": "Ephrin type-A receptor 2",
  "term_id": "GO:0005886"
}